cellular response to aluminum ion [GO:0071275] (BP) Relationships: is a type of GO:0010044; is a type of cellular response to metal ion [GO:0071248] Sources: GOC:mah Definition: Any process that results in a change in state or activity of a cell (in terms of movement, secretion, enzyme production, gene expression, etc.) as a result of an aluminum ion stimulus. Also known as: cellular response to aluminium ion, cellular response to aluminum